septum secundum development [GO:0003285] (biological process) Sources: GOC:mtg_heart Relationships: is a type of atrial septum development [GO:0003283] Definition: The progression of the septum secundum over time, from its initial formation to the mature structure.